{
  "term_label": "aspartate carbamoyltransferase activity",
  "term_id": "GO:0004070",
  "gene_name": "CAD protein",
  "gene_symbol": "CAD",
  "gene": "UniProtKB:P27708"
}